positive regulation of reverse transcription [GO:1900270] (biological process) Sources: GOC:TermGenie Definition: Any process that activates or increases the frequency, rate or extent of reverse transcription. Relationships: is a type of regulation of reverse transcription [GO:1900268]; is a type of GO:2000573; positively regulates reverse transcription [GO:0001171] Also known as: up regulation of reverse transcription, up-regulation of reverse transcription, upregulation of reverse transcription, activation of reverse transcription